{
  "gene_symbol": "FAM167A",
  "term_id": "UNKNOWN:0003",
  "term_label": "Unknown cellular component",
  "gene": "UniProtKB:Q96KS9",
  "gene_name": "Protein FAM167A"
}